{
  "gene_symbol": "SFRP2",
  "term_label": "canonical Wnt signaling pathway",
  "gene_name": "Secreted frizzled-related protein 2",
  "gene": "UniProtKB:Q96HF1",
  "term_id": "GO:0060070"
}